{
  "term_label": "negative regulation of DNA-templated transcription",
  "gene": "UniProtKB:Q9UHJ3",
  "gene_name": "Scm-like with four MBT domains protein 1",
  "gene_symbol": "SFMBT1",
  "term_id": "GO:0045892"
}